telomere maintenance in response to DNA damage [GO:0043247] (biological process) Relationships: is a type of telomere maintenance [GO:0000723]; is a type of DNA damage response [GO:0006974] Subtypes: GO:0031848, telomere maintenance via base-excision repair [GO:0097698] References: PMID:15279784 Sources: GOC:BHF, GOC:BHF_telomere, GOC:jbu Definition: Any process that occur in response to the presence of critically short or damaged telomeres. Also known as: DNA damage response, telomere maintenance Regulation: regulated by regulation of telomere maintenance in response to DNA damage [GO:1904505]; negatively regulated by GO:1904506; positively regulated by GO:1904507